{
  "gene": "UniProtKB:P00738",
  "term_label": "blood microparticle",
  "gene_name": "Haptoglobin",
  "gene_symbol": "HP",
  "term_id": "GO:0072562"
}